{
  "term_label": "NAD(P)H oxidase H2O2-forming activity",
  "gene_symbol": "DUOX1",
  "gene_name": "Dual oxidase 1",
  "term_id": "GO:0016174",
  "gene": "UniProtKB:Q9NRD9"
}